{
  "term_id": "GO:0005737",
  "gene": "UniProtKB:Q7Z406",
  "gene_symbol": "MYH14",
  "gene_name": "Myosin-14",
  "term_label": "cytoplasm"
}